retinal binding [GO:0016918] (molecular function) Subtypes: 11-cis retinal binding [GO:0005502], all-trans retinal binding [GO:0005503] Sources: ISBN:0198506732 Relationships: is a type of retinoid binding [GO:0005501]; is_a vitamin binding [GO:0019842] Also known as: vitamin A binding, retinaldehyde binding, UV-sensitive opsin, blue-sensitive opsin, green-sensitive opsin, long-wave-sensitive opsin, opsin, red-sensitive opsin, short-wave-sensitive opsin, violet-sensitive opsin Definition: Binding to retinal, one of the forms of vitamin A. Retinal plays an important role in the visual process in most vertebrates, combining with opsins to form visual pigments in the retina.